{
  "gene": "UniProtKB:Q13895",
  "term_label": "nucleolus",
  "gene_name": "Bystin",
  "term_id": "GO:0005730",
  "gene_symbol": "BYSL"
}